{
  "term_id": "GO:0000226",
  "gene_name": "MAP7 domain-containing protein 1",
  "gene": "UniProtKB:Q3KQU3",
  "gene_symbol": "MAP7D1",
  "term_label": "microtubule cytoskeleton organization"
}